{
  "gene_name": "Bone morphogenetic protein 3",
  "gene_symbol": "BMP3",
  "term_label": "cytokine activity",
  "term_id": "GO:0005125",
  "gene": "UniProtKB:P12645"
}